{
  "gene_name": "Nociceptin receptor",
  "term_id": "GO:0042923",
  "gene": "UniProtKB:P41146",
  "term_label": "neuropeptide binding",
  "gene_symbol": "OPRL1"
}